{
  "gene": "UniProtKB:Q07837",
  "gene_symbol": "SLC3A1",
  "gene_name": "Neutral and basic amino acid transport protein rBAT",
  "term_id": "UNKNOWN:0001",
  "term_label": "Unknown molecular function"
}